{
  "gene_name": "E3 ubiquitin-protein ligase TRIM11",
  "gene": "UniProtKB:Q96F44",
  "term_label": "negative regulation of viral transcription",
  "term_id": "GO:0032897",
  "gene_symbol": "TRIM11"
}